venom-mediated vasoconstriction via activation of endothelin receptor signaling pathway [GO:0140183] (biological process) Definition: A process in which an organism promotes the narrowing (constriction) of blood vessels, by inhibiting the widening (dilation) of blood vessels in another organism via the action of a venom that activates endothelin receptor signaling pathway, concomittantly increasing blood pressure in the bitten/stung organism. Also known as: venom-mediated vasoconstriction via activation of endothelin signaling pathway, venom-mediated vasoconstriction via activation of endothelin-dependent signaling, venom-mediated vasoconstriction via endothelin receptor agonism Relationships: is a type of venom-mediated activation of G protein-coupled receptor signaling pathway [GO:0044514] References: PMID:16277978